{
  "gene_name": "T-box transcription factor TBX10",
  "term_label": "DNA-binding transcription factor activity, RNA polymerase II-specific",
  "gene": "UniProtKB:O75333",
  "term_id": "GO:0000981",
  "gene_symbol": "TBX10"
}